{
  "term_id": "GO:0005737",
  "gene": "UniProtKB:Q9UET6",
  "gene_symbol": "FTSJ1",
  "gene_name": "Putative tRNA (cytidine(32)_guanosine(34)-2'-O)-methyltransferase",
  "term_label": "cytoplasm"
}